{
  "term_label": "protein maturation",
  "gene": "UniProtKB:O60259",
  "gene_name": "Kallikrein-8",
  "gene_symbol": "KLK8",
  "term_id": "GO:0051604"
}